{
  "term_id": "GO:0008017",
  "term_label": "microtubule binding",
  "gene_name": "Regulator of microtubule dynamics protein 1",
  "gene_symbol": "RMDN1",
  "gene": "UniProtKB:Q96DB5"
}